{
  "term_id": "GO:0004222",
  "gene": "UniProtKB:P09237",
  "gene_symbol": "MMP7",
  "term_label": "metalloendopeptidase activity",
  "gene_name": "Matrilysin"
}